{
  "term_id": "UNKNOWN:0003",
  "gene_symbol": "ITIH1",
  "gene_name": "Inter-alpha-trypsin inhibitor heavy chain H1",
  "term_label": "Unknown cellular component",
  "gene": "UniProtKB:P19827"
}